{
  "gene": "UniProtKB:P0DH78",
  "gene_name": "RING finger protein 224",
  "gene_symbol": "RNF224",
  "term_label": "Unknown molecular function",
  "term_id": "UNKNOWN:0001"
}